{
  "gene": "UniProtKB:P18509",
  "gene_name": "Pituitary adenylate cyclase-activating polypeptide",
  "term_label": "neuron projection development",
  "gene_symbol": "ADCYAP1",
  "term_id": "GO:0031175"
}